{
  "term_label": "postsynaptic density membrane",
  "term_id": "GO:0098839",
  "gene_symbol": "ADAM22",
  "gene": "UniProtKB:Q9P0K1",
  "gene_name": "Disintegrin and metalloproteinase domain-containing protein 22"
}